meiotic sister chromatid cohesion involved in meiosis II [GO:0010790] (biological process) Definition: The cell cycle process in which sister chromatids of a replicated chromosome are joined along the entire length of the chromosome during meiosis II. Relationships: is a type of GO:0051177 Sources: GOC:dph, GOC:tb